{
  "gene_symbol": "IKBKG",
  "gene_name": "NF-kappa-B essential modulator",
  "term_id": "GO:0005634",
  "gene": "UniProtKB:Q9Y6K9",
  "term_label": "nucleus"
}